{
  "term_label": "nucleus",
  "term_id": "GO:0005634",
  "gene_symbol": "SENP1",
  "gene_name": "Sentrin-specific protease 1",
  "gene": "UniProtKB:Q9P0U3"
}